{
  "term_label": "regulation of cellular localization",
  "gene_name": "Partitioning defective 6 homolog gamma",
  "gene": "UniProtKB:Q9BYG4",
  "gene_symbol": "PARD6G",
  "term_id": "GO:0060341"
}